{
  "gene_name": "DNA repair and recombination protein RAD54B",
  "gene_symbol": "RAD54B",
  "gene": "UniProtKB:Q9Y620",
  "term_label": "DNA translocase activity",
  "term_id": "GO:0015616"
}